{
  "term_label": "cytosol",
  "gene": "UniProtKB:C9JCN9",
  "gene_name": "Heat shock factor-binding protein 1-like protein 1",
  "gene_symbol": "HSBP1L1",
  "term_id": "GO:0005829"
}